{
  "term_id": "GO:0006886",
  "gene": "UniProtKB:O75436",
  "term_label": "intracellular protein transport",
  "gene_name": "Vacuolar protein sorting-associated protein 26A",
  "gene_symbol": "VPS26A"
}